{
  "term_label": "actin filament severing",
  "gene": "UniProtKB:O15195",
  "gene_symbol": "VILL",
  "gene_name": "Villin-like protein",
  "term_id": "GO:0051014"
}